{
  "gene_name": "Transcriptional repressor CTCFL",
  "gene": "UniProtKB:Q8NI51",
  "term_id": "GO:0000978",
  "gene_symbol": "CTCFL",
  "term_label": "RNA polymerase II cis-regulatory region sequence-specific DNA binding"
}